{
  "gene_symbol": "MAFA",
  "gene_name": "Transcription factor MafA",
  "term_id": "GO:0000978",
  "term_label": "RNA polymerase II cis-regulatory region sequence-specific DNA binding",
  "gene": "UniProtKB:Q8NHW3"
}